{
  "gene_name": "Serine_threonine-protein kinase SIK1",
  "gene": "UniProtKB:P57059",
  "term_id": "GO:0005737",
  "gene_symbol": "SIK1",
  "term_label": "cytoplasm"
}